{
  "term_id": "UNKNOWN:0002",
  "gene_symbol": "XAGE1B",
  "gene_name": "X antigen family member 1",
  "term_label": "Unknown biological process",
  "gene": "UniProtKB:Q9HD64"
}